C4 photosynthesis [GO:0009760] (biological process) Definition: The combination of atmospheric CO2 with a 3-carbon molecule phosphoenol pyruvate (PEP) in the mesophyll cells to make a 4-carbon acid which is immediately converted to malic acid. The malic acid is then passed across to the bundle sheath cells where it is broken down again to pyruvic acid and CO2. The acid is passed back to the mesophyll cells to be used again, while the CO2 is fed into the reductive pentose-phosphate cycle (Calvin cycle) and converted into sugar and starch. Sources: ISBN:0816017360 Subtypes: NADP-malic enzyme C4 photosynthesis [GO:0009762], NAD-malic enzyme C4 photosynthesis [GO:0009763], PEP carboxykinase C4 photosynthesis [GO:0009764] Relationships: is a type of carbon fixation [GO:0015977]; is a type of photosynthesis, dark reaction [GO:0019685]